lipoprotein biosynthetic process [GO:0042158] (biological process) Definition: The chemical reactions and pathways resulting in the formation of any conjugated, water-soluble protein in which the covalently attached nonprotein group consists of a lipid or lipids. Also known as: lipoprotein anabolism, lipoprotein biosynthesis, lipoprotein formation, lipoprotein synthesis Sources: ISBN:0198506732 Relationships: is a type of macromolecule biosynthetic process [GO:0009059]; is a type of GO:0042157